{
  "term_label": "Unknown molecular function",
  "gene_name": "Mitochondrial import inner membrane translocase subunit TIM50",
  "gene": "UniProtKB:Q3ZCQ8",
  "gene_symbol": "TIMM50",
  "term_id": "UNKNOWN:0001"
}